{
  "term_id": "GO:0008009",
  "gene_name": "Stromal cell-derived factor 1",
  "term_label": "chemokine activity",
  "gene": "UniProtKB:P48061",
  "gene_symbol": "CXCL12"
}